{
  "gene_symbol": "ODAD3",
  "gene_name": "Outer dynein arm-docking complex subunit 3",
  "gene": "UniProtKB:A5D8V7",
  "term_id": "GO:0003341",
  "term_label": "cilium movement"
}